{
  "gene": "UniProtKB:Q6P5W5",
  "gene_symbol": "SLC39A4",
  "term_id": "GO:0071578",
  "term_label": "zinc ion import across plasma membrane",
  "gene_name": "Zinc transporter ZIP4"
}